type-III cohesin domain binding [GO:1990313] (MF) Definition: Binding to a type-III cohesin domain of a protein. Type-III cohesin domain is the binding partner of type-III dockerin domain. References: PMID:23195689, PMID:24080387 Sources: GOC:mengo_curators Relationships: is a type of protein domain specific binding [GO:0019904]